{
  "gene": "UniProtKB:Q5JPI3",
  "term_id": "UNKNOWN:0003",
  "term_label": "Unknown cellular component",
  "gene_name": "Uncharacterized protein C3orf38",
  "gene_symbol": "C3orf38"
}